{
  "gene": "UniProtKB:Q494X3",
  "term_label": "regulation of transcription by RNA polymerase II",
  "term_id": "GO:0006357",
  "gene_name": "Zinc finger protein 404",
  "gene_symbol": "ZNF404"
}